post-embryonic limb morphogenesis [GO:0035127] (BP) Definition: The process, occurring after embryonic development, by which the anatomical structures of the limb are generated and organized. A limb is an appendage of an animal used for locomotion or grasping. Sources: ISBN:0395825172 Relationships: is a type of limb morphogenesis [GO:0035108]; is_a post-embryonic appendage morphogenesis [GO:0035120] Subtypes: post-embryonic forelimb morphogenesis [GO:0035128], GO:0035129